{
  "term_label": "Unknown cellular component",
  "gene_symbol": "NR2C1",
  "term_id": "UNKNOWN:0003",
  "gene_name": "Nuclear receptor subfamily 2 group C member 1",
  "gene": "UniProtKB:P13056"
}